{
  "gene_symbol": "ERBB4",
  "term_id": "GO:0050679",
  "gene_name": "Receptor tyrosine-protein kinase erbB-4",
  "term_label": "positive regulation of epithelial cell proliferation",
  "gene": "UniProtKB:Q15303"
}